{
  "term_label": "regulation of cytokine production",
  "gene_name": "HERV-H LTR-associating protein 2",
  "gene_symbol": "HHLA2",
  "gene": "UniProtKB:Q9UM44",
  "term_id": "GO:0001817"
}